{
  "gene_name": "Roundabout homolog 4",
  "term_id": "GO:0030424",
  "term_label": "axon",
  "gene_symbol": "ROBO4",
  "gene": "UniProtKB:Q8WZ75"
}